{
  "gene_symbol": "LRRC3B",
  "term_id": "GO:0038023",
  "term_label": "signaling receptor activity",
  "gene": "UniProtKB:Q96PB8",
  "gene_name": "Leucine-rich repeat-containing protein 3B"
}